pre-replicative complex assembly [GO:0036388] (biological process) Subtypes: pre-replicative complex assembly involved in cell cycle DNA replication [GO:1902299] Sources: GOC:bf, GOC:bhm, GOC:jh2 Also known as: pre-RC assembly, pre-replication complex assembly Definition: The aggregation, arrangement and bonding together of a set of components to form the pre-replicative complex, a protein-DNA complex that forms at the origin of replication during the initial step of DNA replication and allows the origin to become competent, or 'licensed', for replication. Relationships: is a type of protein-DNA complex assembly [GO:0065004]; BFO_0000050 DNA-templated DNA replication [GO:0006261]